inosine transport [GO:0035340] (biological process) Definition: The directed movement of the purine ribonucleoside inosine, also known as hypoxanthine riboside, into, out of or within a cell, or between cells, by means of some agent such as a transporter or pore. Also known as: hypoxanthine riboside transport References: PMID:19135251 Regulation: regulated by GO:0035341; positively regulated by GO:0035342; negatively regulated by negative regulation of inosine transport [GO:0035343] Relationships: is a type of nucleoside transport [GO:0015858]